{
  "gene_symbol": "MBIP",
  "gene_name": "MAP3K12-binding inhibitory protein 1",
  "gene": "UniProtKB:Q9NS73",
  "term_id": "UNKNOWN:0002",
  "term_label": "Unknown biological process"
}